{
  "gene_symbol": "CHRNB3",
  "gene": "UniProtKB:Q05901",
  "gene_name": "Neuronal acetylcholine receptor subunit beta-3",
  "term_id": "GO:0022848",
  "term_label": "acetylcholine-gated monoatomic cation-selective channel activity"
}